{
  "term_label": "potassium ion transmembrane transport",
  "gene_symbol": "KCNH4",
  "gene_name": "Potassium voltage-gated channel subfamily H member 4",
  "gene": "UniProtKB:Q9UQ05",
  "term_id": "GO:0071805"
}